{
  "term_id": "GO:0005789",
  "gene_name": "Transmembrane 6 superfamily member 2",
  "gene_symbol": "TM6SF2",
  "term_label": "endoplasmic reticulum membrane",
  "gene": "UniProtKB:Q9BZW4"
}